{
  "gene_name": "Target of EGR1 protein 1",
  "gene": "UniProtKB:Q96GM8",
  "gene_symbol": "TOE1",
  "term_id": "GO:0015030",
  "term_label": "Cajal body"
}